gemmule [GO:0097463] (cellular component) Sources: NIF_Subcellular:nlx_subcell_1005003 Relationships: is_a neuron projection [GO:0043005] Definition: Spine-like process found on some neurons, e.g., periglomerular cells of olfactory cortex.